smoothened signaling pathway [GO:0007224] (BP) Definition: The series of molecular signals generated as a consequence of activation of the transmembrane protein Smoothened. Regulation: regulated by regulation of smoothened signaling pathway [GO:0008589]; negatively regulated by GO:0045879; positively regulated by positive regulation of smoothened signaling pathway [GO:0045880] References: PMID:15057936, PMID:15205520 Sources: GOC:mah Also known as: hedgehog signaling pathway, smoothened signalling pathway, Sonic hedgehog signaling pathway, hh signaling pathway, hh signalling pathway, Shh signaling pathway Relationships: is a type of cell surface receptor signaling pathway [GO:0007166] Subtypes: GO:0003271, smoothened signaling pathway involved in ventral spinal cord patterning [GO:0021910], smoothened signaling pathway involved in regulation of cerebellar granule cell precursor cell proliferation [GO:0021938], smoothened signaling pathway involved in lung development [GO:0060506], mesenchymal smoothened signaling pathway involved in prostate gland development [GO:0060783], GO:0060831